scopoletin 8-hydroxylase activity [GO:0106145] (molecular function) Relationships: is a type of oxidoreductase activity, acting on paired donors, with incorporation or reduction of molecular oxygen, NAD(P)H as one donor, and incorporation of one atom of oxygen [GO:0016709] Definition: Catalyzes of the reaction: scopoletin + 2-oxoglutarate+O2=fraxetin +succinate+ CO2). References: PMID:29361149, PMID:29581584 Sources: GOC:lr, RHEA:57848